MAML2-RBP-Jkappa-ICN2 complex [GO:0071176] (cellular component) Also known as: MAML2-RBP-Jkappa-Notch2 complex Definition: A protein complex that consists of the intracellular domain of Notch2 (ICN2), the DNA-binding transcription factor RBP-Jkappa, and the transcriptional coactivator Mastermind-like-2 (MAML2); the complex is involved in transcriptional activation in response to Notch-mediated signaling. Relationships: is a type of nuclear protein-containing complex [GO:0140513] References: PMID:12370315